{
  "term_id": "GO:0001669",
  "gene": "UniProtKB:P04279",
  "gene_name": "Semenogelin-1",
  "term_label": "acrosomal vesicle",
  "gene_symbol": "SEMG1"
}